{
  "gene_symbol": "LINC00596",
  "term_id": "UNKNOWN:0001",
  "term_label": "Unknown molecular function",
  "gene": "UniProtKB:Q86U02",
  "gene_name": "Putative uncharacterized protein encoded by LINC00596"
}